dehydroquinate synthase activity [GO:0102042] (molecular function) Definition: Catalysis of the reaction: 2-amino-2,3,7-trideoxy-D-lyxo-hept-6-ulosonic acid + H2O + NAD = 3-dehydroquinate + ammonium + NADH + H+. Sources: GOC:pz, RHEA:25956 Relationships: is a type of oxidoreductase activity, acting on the CH-NH2 group of donors, NAD or NADP as acceptor [GO:0016639]